{
  "term_label": "cytoplasm",
  "gene_symbol": "CPOX",
  "gene_name": "Oxygen-dependent coproporphyrinogen-III oxidase, mitochondrial",
  "term_id": "GO:0005737",
  "gene": "UniProtKB:P36551"
}